{
  "gene": "UniProtKB:Q15019",
  "term_label": "intracellular protein localization",
  "gene_name": "Septin-2",
  "gene_symbol": "SEPTIN2",
  "term_id": "GO:0008104"
}